{
  "gene_symbol": "DR1",
  "term_label": "RNA polymerase II general transcription initiation factor activity",
  "gene": "UniProtKB:Q01658",
  "gene_name": "Protein Dr1",
  "term_id": "GO:0016251"
}